{
  "term_label": "membrane",
  "gene_name": "Starch-binding domain-containing protein 1",
  "term_id": "GO:0016020",
  "gene": "UniProtKB:O95210",
  "gene_symbol": "STBD1"
}